{
  "term_label": "mitochondrial respiratory chain complex IV assembly",
  "gene_symbol": "COX14",
  "gene_name": "Cytochrome c oxidase assembly protein COX14",
  "gene": "UniProtKB:Q96I36",
  "term_id": "GO:0033617"
}